{
  "gene_symbol": "PCDHA2",
  "term_id": "GO:0005886",
  "term_label": "plasma membrane",
  "gene": "UniProtKB:Q9Y5H9",
  "gene_name": "Protocadherin alpha-2"
}